{
  "term_label": "cAMP binding",
  "gene_symbol": "PRKAR1A",
  "gene_name": "cAMP-dependent protein kinase type I-alpha regulatory subunit",
  "term_id": "GO:0030552",
  "gene": "UniProtKB:P10644"
}